regulation of mammary gland cord elongation by mammary fat precursor cell-epithelial cell signaling [GO:0060657] (biological process) Relationships: is a type of cell-cell signaling [GO:0007267]; is a type of regulation of developmental growth [GO:0048638]; regulates mammary gland cord elongation [GO:0060654] Also known as: regulation of mammary gland cord elongation by mammary fat precursor cell-epithelial cell signalling Definition: Any process that modulates the rate, frequency, or extent of mammary gland cord elongation as a result of a signal being created by a mesenchymal cell that is a precursor to the mammary fat and its subsequent reception and interpretation by an mammary cord epithelial cell. References: PMID:12558599 Sources: GOC:dph